{
  "term_id": "GO:0048018",
  "gene_name": "C-type lectin domain family 2 member D",
  "gene_symbol": "CLEC2D",
  "term_label": "receptor ligand activity",
  "gene": "UniProtKB:Q9UHP7"
}